{
  "gene": "UniProtKB:Q8NE71",
  "term_label": "Unknown cellular component",
  "term_id": "UNKNOWN:0003",
  "gene_name": "ATP-binding cassette sub-family F member 1",
  "gene_symbol": "ABCF1"
}